{
  "term_label": "Unknown cellular component",
  "gene": "UniProtKB:Q16769",
  "term_id": "UNKNOWN:0003",
  "gene_name": "Glutaminyl-peptide cyclotransferase",
  "gene_symbol": "QPCT"
}